{
  "term_id": "GO:0007030",
  "gene_symbol": "GOLGA8H",
  "gene": "UniProtKB:P0CJ92",
  "gene_name": "Golgin subfamily A member 8H",
  "term_label": "Golgi organization"
}